{
  "term_label": "neuron differentiation",
  "gene_name": "LIM homeobox transcription factor 1-beta",
  "gene": "UniProtKB:O60663",
  "gene_symbol": "LMX1B",
  "term_id": "GO:0030182"
}